myosin VI head/neck binding [GO:0070855] (molecular function) Relationships: is a type of myosin head/neck binding [GO:0032028]; is a type of myosin VI heavy chain binding [GO:0070854] Sources: GOC:sart Definition: Binding to the head/neck region of a myosin VI heavy chain.